{
  "gene_name": "Glutathione hydrolase 1 proenzyme",
  "gene": "UniProtKB:P19440",
  "gene_symbol": "GGT1",
  "term_label": "glutathione catabolic process",
  "term_id": "GO:0006751"
}